regulation of nuclear migration during mitotic telophase [GO:1902852] (biological process) References: PMID:23087209 Sources: GOC:TermGenie, GO_REF:0000058 Subtypes: negative regulation of nuclear migration during mitotic telophase [GO:1902853], GO:1902854 Definition: Any process that modulates the frequency, rate or extent of nuclear migration during mitotic telophase. Relationships: is a type of GO:1902838; RO_0002211 nuclear migration during mitotic telophase [GO:0090561]